{
  "term_label": "endoplasmic reticulum membrane",
  "gene": "UniProtKB:Q9C0D9",
  "gene_symbol": "SELENOI",
  "term_id": "GO:0005789",
  "gene_name": "Ethanolaminephosphotransferase 1"
}